gluconate 5-dehydrogenase activity [GO:0008874] (molecular function) Sources: EC:1.1.1.69 Definition: Catalysis of the reaction: D-gluconate + NADP+ = 5-dehydro-D-gluconate + NADPH + H+. Also known as: 5-keto-D-gluconate 5-reductase activity, 5-keto-D-gluconate reductase, 5-ketogluconate 5-reductase activity, 5-ketogluconate reductase activity, D-gluconate:NAD(P)+ 5-oxidoreductase Relationships: is a type of gluconate dehydrogenase activity [GO:0008875]